{
  "gene_name": "Transcription factor YY2",
  "gene_symbol": "YY2",
  "gene": "UniProtKB:O15391",
  "term_label": "transcription regulator complex",
  "term_id": "GO:0005667"
}